{
  "gene_symbol": "MRGPRG",
  "term_label": "G protein-coupled receptor activity",
  "gene_name": "Mas-related G-protein coupled receptor member G",
  "gene": "UniProtKB:Q86SM5",
  "term_id": "GO:0004930"
}